{
  "term_label": "regulation of protein stability",
  "gene_name": "Probable ubiquitin carboxyl-terminal hydrolase FAF-Y",
  "gene_symbol": "USP9Y",
  "gene": "UniProtKB:O00507",
  "term_id": "GO:0031647"
}